{
  "gene_symbol": "RPL27A",
  "gene": "UniProtKB:P46776",
  "term_id": "GO:0003735",
  "gene_name": "Large ribosomal subunit protein uL15",
  "term_label": "structural constituent of ribosome"
}